{
  "gene_symbol": "CMYA5",
  "gene": "UniProtKB:Q8N3K9",
  "gene_name": "Cardiomyopathy-associated protein 5",
  "term_id": "UNKNOWN:0002",
  "term_label": "Unknown biological process"
}